positive regulation of MyD88-independent toll-like receptor signaling pathway [GO:0034129] (biological process) References: PMID:16551253, PMID:17328678 Sources: GOC:add Relationships: is a type of GO:0034123; is_a regulation of MyD88-independent toll-like receptor signaling pathway [GO:0034127]; RO_0002213 GO:0002756 Definition: Any process that activates or increases the frequency, rate, or extent of MyD88-independent toll-like receptor signaling pathway. Also known as: positive regulation of MyD88-independent TLR signaling pathway, positive regulation of MyD88-independent toll-like receptor, positive regulation of MyD88-independent toll-like receptor signalling pathway